cell dedifferentiation involved in phenotypic switching [GO:0090678] (biological process) Sources: GOC:curators Definition: A cell dedifferentiation process that is a part of a reversible switch of a cell from one cell type or form to another, at a frequency above the expected frequency for somatic mutations. Relationships: is a type of cell dedifferentiation [GO:0043697]; is part of reversible differentiation [GO:0090677] Subtypes: vascular associated smooth muscle cell dedifferentiation [GO:1990936]